{
  "term_label": "ubiquitin protein ligase activity",
  "term_id": "GO:0061630",
  "gene": "UniProtKB:E7ERA6",
  "gene_name": "RING finger protein 223",
  "gene_symbol": "RNF223"
}